response to methamphetamine hydrochloride [GO:1904313] (biological process) Relationships: is a type of GO:0014075 Definition: Any process that results in a change in state or activity of a cell or an organism (in terms of movement, secretion, enzyme production, gene expression, etc.) as a result of a methamphetamine hydrochloride stimulus. References: PMID:22174933 Sources: GOC:TermGenie, GO_REF:0000071 Also known as: response to methamphetamine HCL Subtypes: cellular response to methamphetamine hydrochloride [GO:1904314]